{
  "gene_symbol": "YTHDF2",
  "gene_name": "YTH domain-containing family protein 2",
  "term_label": "cytoplasm",
  "gene": "UniProtKB:Q9Y5A9",
  "term_id": "GO:0005737"
}